{
  "gene_name": "Methyltransferase-like protein 25B",
  "gene_symbol": "METTL25B",
  "term_id": "UNKNOWN:0002",
  "gene": "UniProtKB:Q96FB5",
  "term_label": "Unknown biological process"
}